{
  "gene_symbol": "IGLJ7",
  "term_label": "Unknown biological process",
  "gene": "UniProtKB:A0A0A0MT92",
  "term_id": "UNKNOWN:0002",
  "gene_name": "Immunoglobulin lambda joining 7 (Fragment)"
}